{
  "gene_symbol": "ONECUT2",
  "gene": "UniProtKB:O95948",
  "term_id": "GO:0000978",
  "gene_name": "One cut domain family member 2",
  "term_label": "RNA polymerase II cis-regulatory region sequence-specific DNA binding"
}